{
  "gene": "UniProtKB:Q7Z5Q1",
  "term_id": "GO:0005737",
  "term_label": "cytoplasm",
  "gene_symbol": "CPEB2",
  "gene_name": "Cytoplasmic polyadenylation element-binding protein 2"
}